{
  "term_label": "acyl-CoA metabolic process",
  "gene_symbol": "ACOT11",
  "gene": "UniProtKB:Q8WXI4",
  "gene_name": "Acyl-coenzyme A thioesterase 11",
  "term_id": "GO:0006637"
}